tRNA m2,2-guanine biosynthesis [GO:0002942] (biological process) Relationships: is a type of tRNA methylation [GO:0030488] Sources: GOC:hjd, ISBN:155581073X Definition: The process whereby a guanine residue in a transfer RNA is methylated twice at the N2 position.